{
  "gene": "UniProtKB:Q5XKR4",
  "term_label": "DNA binding",
  "gene_name": "Homeobox protein orthopedia",
  "gene_symbol": "OTP",
  "term_id": "GO:0003677"
}